basement membrane disassembly involved in semicircular canal fusion [GO:0060882] (biological process) Relationships: is a type of basement membrane disassembly [GO:0034769]; is part of semicircular canal fusion [GO:0060879] Sources: GOC:dph, GOC:sdb_2009, GOC:tb Definition: A process that results in the breakdown of the basement membrane that contributes to the process of semicircular canal fusion. Also known as: basal lamina disassembly involved in semicircular canal fusion